{
  "term_id": "GO:1902711",
  "gene_symbol": "GABRB2",
  "gene_name": "Gamma-aminobutyric acid receptor subunit beta-2",
  "gene": "UniProtKB:P47870",
  "term_label": "GABA-A receptor complex"
}